{
  "gene": "UniProtKB:Q9BXW9",
  "term_id": "GO:0000793",
  "gene_name": "Fanconi anemia group D2 protein",
  "term_label": "condensed chromosome",
  "gene_symbol": "FANCD2"
}